type 1 melanocortin receptor binding [GO:0070996] (molecular function) Relationships: is a type of melanocortin receptor binding [GO:0031779] Definition: Binding to a type 1 melanocortin receptor. Sources: GOC:BHF, GOC:mah Also known as: type 1 melanocortin receptor ligand